{
  "gene_name": "Cytochrome P450 1A1",
  "gene": "UniProtKB:P04798",
  "gene_symbol": "CYP1A1",
  "term_label": "estrogen metabolic process",
  "term_id": "GO:0008210"
}